{
  "gene_symbol": "MRPL17",
  "gene": "UniProtKB:Q9NRX2",
  "term_id": "GO:0005762",
  "gene_name": "Large ribosomal subunit protein bL17m",
  "term_label": "mitochondrial large ribosomal subunit"
}